{
  "gene_name": "NEDD4-binding protein 2-like 2",
  "term_id": "GO:0000122",
  "gene_symbol": "N4BP2L2",
  "term_label": "negative regulation of transcription by RNA polymerase II",
  "gene": "UniProtKB:Q92802"
}